{
  "gene_symbol": "NKPD1",
  "gene_name": "NTPase KAP family P-loop domain-containing protein 1",
  "gene": "UniProtKB:Q17RQ9",
  "term_label": "Unknown biological process",
  "term_id": "UNKNOWN:0002"
}